{
  "gene_symbol": "SPMIP10",
  "gene": "UniProtKB:Q6ZNM6",
  "term_label": "Unknown molecular function",
  "gene_name": "Testis-expressed protein 43",
  "term_id": "UNKNOWN:0001"
}